sodium-dependent self proteolysis [GO:1990091] (biological process) Definition: The sodium-dependent hydrolysis of proteins into smaller polypeptides and/or amino acids by cleavage of their own peptide bonds. Relationships: is a type of self proteolysis [GO:0097264] References: PMID:20460380